{
  "term_id": "UNKNOWN:0001",
  "term_label": "Unknown molecular function",
  "gene_symbol": "KIFAP3",
  "gene": "UniProtKB:Q92845",
  "gene_name": "Kinesin-associated protein 3"
}